{
  "gene": "UniProtKB:O15165",
  "term_label": "R-SMAD binding",
  "gene_symbol": "LDLRAD4",
  "term_id": "GO:0070412",
  "gene_name": "Low-density lipoprotein receptor class A domain-containing protein 4"
}